NAD+ catabolic process [GO:0019677] (biological process) Definition: The chemical reactions and pathways resulting in the breakdown of nicotinamide adenine dinucleotide (NAD+), a coenzyme that interconverts with its reduced form, NADH, in many redox and catabolic reactions. References: PMID:28648096 Relationships: is a type of purine nucleotide catabolic process [GO:0006195]; is a type of pyridine nucleotide catabolic process [GO:0019364]; is a type of NAD+ metabolic process [GO:0019674] Also known as: NAD (oxidized) catabolic process, NAD (oxidized) catabolism, NAD (reduced) catabolic process, NAD (reduced) catabolism, NAD breakdown, NAD catabolic process, NAD catabolism, NAD degradation, NADH catabolic process, NADH catabolism, nicotinamide adenine dinucleotide catabolic process, nicotinamide adenine dinucleotide catabolism, oxidized NAD catabolic process, oxidized NAD catabolism, oxidized nicotinamide adenine dinucleotide catabolic process, oxidized nicotinamide adenine dinucleotide catabolism, reduced NAD catabolic process, reduced NAD catabolism, reduced nicotinamide adenine dinucleotide catabolic process, reduced nicotinamide adenine dinucleotide catabolism